{
  "gene": "UniProtKB:Q9P2N7",
  "term_label": "Cul3-RING ubiquitin ligase complex",
  "gene_name": "Kelch-like protein 13",
  "term_id": "GO:0031463",
  "gene_symbol": "KLHL13"
}